{
  "gene": "UniProtKB:Q15617",
  "gene_symbol": "OR8G1",
  "term_label": "odorant binding",
  "term_id": "GO:0005549",
  "gene_name": "Olfactory receptor 8G1"
}